glycosaminoglycan galactosyltransferase activity [GO:0047271] (MF) Sources: EC:2.4.1.74, MetaCyc:2.4.1.74-RXN Relationships: is a type of UDP-galactosyltransferase activity [GO:0035250] Also known as: UDP-galactose:glycosaminoglycan D-galactosyltransferase activity, UDPgalactose:glycosaminoglycan D-galactosyltransferase activity, uridine diphosphogalactose-mucopolysaccharide galactosyltransferase activity Definition: Catalysis of the reaction: glycosaminoglycan + UDP-galactose = D-galactosylglycosaminoglycan + UDP.